positive regulation of methane biosynthetic process from 3-(methylthio)propionic acid [GO:1900335] (biological process) Also known as: up regulation of methane biosynthetic process from 3-(methylthio)propionic acid, up-regulation of methane biosynthetic process from 3-(methylthio)propionic acid, upregulation of methane biosynthetic process from 3-(methylthio)propionic acid, activation of methane biosynthetic process from 3-(methylthio)propionic acid Sources: GOC:TermGenie, GOC:mengo_curators Definition: Any process that activates or increases the frequency, rate or extent of methane biosynthetic process from 3-(methylthio)propionic acid. Relationships: is a type of positive regulation of fatty acid metabolic process [GO:0045923]; is a type of regulation of methane biosynthetic process from 3-(methylthio)propionic acid [GO:1900333]; is a type of GO:1901579; is a type of positive regulation of cellular respiration [GO:1901857]; positively regulates GO:2001132